{
  "gene_name": "Surfeit locus protein 6",
  "gene_symbol": "SURF6",
  "term_label": "ribosomal small subunit biogenesis",
  "gene": "UniProtKB:O75683",
  "term_id": "GO:0042274"
}